{
  "gene_symbol": "DTYMK",
  "gene": "UniProtKB:P23919",
  "gene_name": "Thymidylate kinase",
  "term_label": "dTTP biosynthetic process",
  "term_id": "GO:0006235"
}